cyclohexyl-isocyanide hydratase activity [GO:0050549] (molecular function) Relationships: is a type of hydro-lyase activity [GO:0016836] Sources: EC:4.2.1.103, RHEA:18197 Definition: Catalysis of the reaction: N-cyclohexylformamide + H+ = cyclohexyl isocyanide + H2O. Also known as: N-cyclohexylformamide hydro-lyase (cyclohexyl-isocyanide-forming), N-cyclohexylformamide hydro-lyase activity, isonitrile hydratase activity